{
  "gene_name": "Protocadherin-9",
  "gene": "UniProtKB:Q9HC56",
  "term_label": "cell adhesion molecule binding",
  "gene_symbol": "PCDH9",
  "term_id": "GO:0050839"
}